glutamine-fructose-6-phosphate transaminase (isomerizing) activity [GO:0004360] (molecular function) Also known as: glucosaminephosphate isomerase, glucosamine-6-phosphate isomerase (glutamine-forming) activity, D-fructose-6-phosphate amidotransferase activity, GlcN6P synthase activity, L-glutamine-D-fructose-6-phosphate amidotransferase activity, L-glutamine:D-fructose-6-phosphate isomerase (deaminating), glucosamine 6-phosphate synthase activity, glucosamine--fructose-6-phosphate aminotransferase (isomerizing) activity, glucosamine-6-phosphate synthase activity, hexosephosphate aminotransferase activity Definition: Catalysis of the reaction: beta-D-fructose 6-phosphate + L-glutamine = D-glucosamine 6-phosphate + L-glutamate. Relationships: is_a GO:0070548 Sources: EC:2.6.1.16, RHEA:13237